protein localization to septin ring [GO:1902935] (biological process) Definition: A process in which a protein is transported to, or maintained in, a location within a septin ring. Relationships: is a type of protein localization to cytoskeleton [GO:0044380]; is a type of protein localization to cell cortex [GO:0072697] References: PMID:16325501 Sources: GOC:TermGenie, GO_REF:0000087 Also known as: protein localisation in septin ring, protein localisation to septin ring, protein localization in septin ring